{
  "gene": "UniProtKB:P0C5Z0",
  "term_id": "GO:0030527",
  "gene_symbol": "H2AB3",
  "term_label": "structural constituent of chromatin",
  "gene_name": "Histone H2A-Bbd type 2_3"
}